{
  "gene_name": "Anion exchange transporter",
  "term_label": "oxalate transmembrane transporter activity",
  "gene_symbol": "SLC26A7",
  "gene": "UniProtKB:Q8TE54",
  "term_id": "GO:0019531"
}